{
  "term_id": "GO:0034703",
  "term_label": "cation channel complex",
  "gene_name": "Short transient receptor potential channel 7",
  "gene": "UniProtKB:Q9HCX4",
  "gene_symbol": "TRPC7"
}